{
  "term_id": "GO:0005829",
  "term_label": "cytosol",
  "gene_name": "Spindlin-4",
  "gene": "UniProtKB:Q56A73",
  "gene_symbol": "SPIN4"
}